{
  "gene_symbol": "TFPT",
  "gene_name": "TCF3 fusion partner",
  "term_id": "GO:0031011",
  "gene": "UniProtKB:P0C1Z6",
  "term_label": "Ino80 complex"
}